{
  "gene_symbol": "SPPL3",
  "term_label": "membrane protein proteolysis",
  "term_id": "GO:0033619",
  "gene": "UniProtKB:Q8TCT6",
  "gene_name": "Signal peptide peptidase-like 3"
}